{
  "gene_name": "Olfactory receptor 2M2",
  "term_id": "GO:0005886",
  "gene": "UniProtKB:Q96R28",
  "gene_symbol": "OR2M2",
  "term_label": "plasma membrane"
}